{
  "term_id": "GO:0001580",
  "term_label": "detection of chemical stimulus involved in sensory perception of bitter taste",
  "gene": "UniProtKB:Q9NYW7",
  "gene_symbol": "TAS2R1",
  "gene_name": "Taste receptor type 2 member 1"
}